{
  "gene_symbol": "GOLGA1",
  "term_label": "Unknown molecular function",
  "term_id": "UNKNOWN:0001",
  "gene": "UniProtKB:Q92805",
  "gene_name": "Golgin subfamily A member 1"
}